{
  "gene": "UniProtKB:A0A6Q8PFD8",
  "term_id": "UNKNOWN:0001",
  "gene_name": "Uncharacterized protein",
  "gene_symbol": "A0A6Q8PFD8",
  "term_label": "Unknown molecular function"
}